{
  "gene_name": "Exosome complex component RRP42",
  "term_id": "GO:0034475",
  "term_label": "U4 snRNA 3'-end processing",
  "gene": "UniProtKB:Q15024",
  "gene_symbol": "EXOSC7"
}